protein-heme linkage [GO:0017003] (biological process) Definition: The covalent linkage of heme and a protein. Sources: GOC:ma Also known as: protein-haem linkage Relationships: is a type of protein-tetrapyrrole linkage [GO:0017006] Subtypes: cytochrome c-heme linkage [GO:0018063], protein-heme P460 linkage [GO:0018174], GO:0018186